{
  "gene_symbol": "PRELID1",
  "term_id": "GO:0005758",
  "term_label": "mitochondrial intermembrane space",
  "gene": "UniProtKB:Q9Y255",
  "gene_name": "PRELI domain-containing protein 1, mitochondrial"
}